{
  "term_label": "NAD+ poly-ADP-ribosyltransferase activity",
  "gene": "UniProtKB:O95271",
  "gene_symbol": "TNKS",
  "term_id": "GO:0003950",
  "gene_name": "Poly [ADP-ribose] polymerase tankyrase-1"
}